{
  "gene": "UniProtKB:P43034",
  "gene_symbol": "PAFAH1B1",
  "term_label": "vesicle transport along microtubule",
  "term_id": "GO:0047496",
  "gene_name": "Platelet-activating factor acetylhydrolase IB subunit beta"
}